{
  "gene_symbol": "KCNA2",
  "gene": "UniProtKB:P16389",
  "term_id": "GO:0016020",
  "gene_name": "Potassium voltage-gated channel subfamily A member 2",
  "term_label": "membrane"
}